{
  "term_id": "GO:0005886",
  "term_label": "plasma membrane",
  "gene_symbol": "IL1RAPL1",
  "gene_name": "Interleukin-1 receptor accessory protein-like 1",
  "gene": "UniProtKB:Q9NZN1"
}